DNA strand elongation involved in premeiotic DNA replication [GO:1902982] (biological process) Definition: Any DNA strand elongation involved in meiotic cell cycle DNA replication. Sources: GOC:TermGenie, GO_REF:0000060 Also known as: DNA strand elongation involved in meiotic cell cycle DNA replication Relationships: is a type of DNA strand elongation involved in nuclear cell cycle DNA replication [GO:1902319]; is a type of meiotic cell cycle process [GO:1903046]; is part of premeiotic DNA replication [GO:0006279]